{
  "gene_name": "TSSK6-activating co-chaperone protein",
  "gene": "UniProtKB:Q96A04",
  "term_id": "UNKNOWN:0002",
  "gene_symbol": "TSACC",
  "term_label": "Unknown biological process"
}